{
  "term_id": "GO:0050776",
  "gene": "UniProtKB:Q92835",
  "gene_name": "Phosphatidylinositol 3,4,5-trisphosphate 5-phosphatase 1",
  "gene_symbol": "INPP5D",
  "term_label": "regulation of immune response"
}